cellotriose catabolic process [GO:2000894] (biological process) Also known as: cellotriose catabolism Definition: The chemical reactions and pathways resulting in the breakdown of a cellotriose. Sources: GOC:mengo_curators Relationships: is a type of oligosaccharide catabolic process [GO:0009313]; is a type of cellotriose metabolic process [GO:2000893] Regulation: regulated by GO:2000936; negatively regulated by negative regulation of cellotriose catabolic process [GO:2000937]; RO_0002213 by GO:2000938